pancreatic PP cell differentiation [GO:0003312] (biological process) Definition: The process in which relatively unspecialized cells acquire specialized structural and functional features of a pancreatic polypeptide-producing cell. A pancreatic polypeptide-producing cell is a cell in the pancreas that produces pancreatic polypeptide. Also known as: pancreatic polypeptide-producing cell differentiation References: PMID:11076772 Sources: GOC:dph Relationships: is a type of GO:0035883; is part of endocrine pancreas development [GO:0031018]